{
  "gene_symbol": "CDYL2",
  "term_label": "transcription corepressor activity",
  "gene": "UniProtKB:Q8N8U2",
  "term_id": "GO:0003714",
  "gene_name": "Chromodomain Y-like protein 2"
}